{
  "term_label": "mitochondrial matrix",
  "gene_name": "Acyl-coenzyme A synthetase ACSM4, mitochondrial",
  "gene_symbol": "ACSM4",
  "gene": "UniProtKB:P0C7M7",
  "term_id": "GO:0005759"
}